viral protein processing [GO:0019082] (biological process) Sources: GOC:bf, GOC:jl, ISBN:0781702534 Relationships: is a type of viral process [GO:0016032]; is part of GO:0019080 Definition: Any protein maturation process achieved by the cleavage of a peptide bond or bonds within a viral protein.